{
  "gene_name": "Potassium voltage-gated channel subfamily E member 2",
  "gene_symbol": "KCNE2",
  "gene": "UniProtKB:Q9Y6J6",
  "term_id": "GO:0086011",
  "term_label": "membrane repolarization during action potential"
}